{
  "term_label": "endomembrane system",
  "gene": "UniProtKB:Q9BWS9",
  "gene_symbol": "CHID1",
  "gene_name": "Chitinase domain-containing protein 1",
  "term_id": "GO:0012505"
}